{
  "term_id": "UNKNOWN:0002",
  "gene": "UniProtKB:Q8WUJ1",
  "gene_name": "Neuferricin",
  "gene_symbol": "CYB5D2",
  "term_label": "Unknown biological process"
}